{
  "gene_name": "Testis-expressed protein 10",
  "term_label": "Unknown molecular function",
  "term_id": "UNKNOWN:0001",
  "gene_symbol": "TEX10",
  "gene": "UniProtKB:Q9NXF1"
}